{
  "gene_symbol": "MRPS14",
  "term_label": "mitochondrial small ribosomal subunit",
  "gene_name": "Small ribosomal subunit protein uS14m",
  "gene": "UniProtKB:O60783",
  "term_id": "GO:0005763"
}